P2Y1 nucleotide receptor binding [GO:0031812] (molecular function) Also known as: P2Y1 nucleotide receptor ligand Definition: Binding to a P2Y1 nucleotide receptor. Relationships: is a type of G protein-coupled nucleotide receptor binding [GO:0031811] Sources: GOC:mah, GOC:nln